{
  "term_id": "GO:0005658",
  "gene": "UniProtKB:P49643",
  "gene_symbol": "PRIM2",
  "gene_name": "DNA primase large subunit",
  "term_label": "alpha DNA polymerase:primase complex"
}